{
  "gene_symbol": "FIGNL1",
  "gene_name": "Fidgetin-like protein 1",
  "gene": "UniProtKB:Q6PIW4",
  "term_id": "GO:0005737",
  "term_label": "cytoplasm"
}